regulation of coenzyme F420-dependent bicyclic nitroimidazole catabolic process [GO:1900288] (biological process) Sources: GOC:TermGenie, GOC:mengo_curators Also known as: regulation of coenzyme F420-dependent nitroimidazole breakdown, regulation of coenzyme F420-dependent nitroimidazole catabolism, regulation of coenzyme F420-dependent nitroimidazole reduction, regulation of coenzyme F420-dependent nitroreductase activity Relationships: is a type of regulation of catabolic process [GO:0009894]; regulates GO:0052799 Definition: Any process that modulates the frequency, rate or extent of coenzyme F420-dependent bicyclic nitroimidazole catabolic process. Subtypes: negative regulation of coenzyme F420-dependent bicyclic nitroimidazole catabolic process [GO:1900289], positive regulation of coenzyme F420-dependent bicyclic nitroimidazole catabolic process [GO:1900290]